{
  "gene_name": "Endoplasmic reticulum resident protein 44",
  "gene": "UniProtKB:Q9BS26",
  "term_id": "GO:0005789",
  "term_label": "endoplasmic reticulum membrane",
  "gene_symbol": "ERP44"
}